{
  "gene_name": "Large ribosomal subunit protein bL17m",
  "gene": "UniProtKB:Q9NRX2",
  "gene_symbol": "MRPL17",
  "term_id": "GO:0003735",
  "term_label": "structural constituent of ribosome"
}